meiotic nuclear membrane microtubule tethering complex [GO:0034993] (cellular component) Definition: A nuclear membrane protein complex which connects the nuclear outer and inner membranes together, and links links the nuclear lumen to cytoplasmic microtubules during meiosis. References: PMID:18692466 Sources: GOC:mah Relationships: is a type of nuclear membrane microtubule tethering complex [GO:0106094]; is part of microtubule organizing center attachment site [GO:0034992] Subtypes: GO:1990612 Also known as: LINC complex, LInker of Nucleoskeleton and Cytoskeleton complex, SUN-KASH complex